{
  "gene_name": "COP9 signalosome complex subunit 5",
  "term_id": "GO:0005737",
  "gene_symbol": "COPS5",
  "gene": "UniProtKB:Q92905",
  "term_label": "cytoplasm"
}